{
  "term_label": "ubiquitin protein ligase activity",
  "gene": "UniProtKB:A0A2R8Y4M4",
  "term_id": "GO:0061630",
  "gene_symbol": "LOC122513141",
  "gene_name": "RING-type domain-containing protein"
}